{
  "term_id": "GO:0005615",
  "gene_symbol": "C4B_2",
  "gene_name": "Complement C4-B",
  "term_label": "extracellular space",
  "gene": "UniProtKB:P0C0L5"
}